positive regulation of cell migration [GO:0030335] (biological process) Subtypes: GO:0002687, GO:0010595, positive regulation of epithelial cell migration [GO:0010634], positive regulation of fibroblast migration [GO:0010763], positive regulation of smooth muscle cell migration [GO:0014911], positive regulation of cell migration by vascular endothelial growth factor signaling pathway [GO:0038089], positive regulation of neuroblast migration [GO:0061854], positive regulation of myotube cell migration [GO:0110124], positive regulation of trophoblast cell migration [GO:1901165], positive regulation of distal tip cell migration [GO:1903356], positive regulation of wound healing, spreading of epidermal cells [GO:1903691], positive regulation of glial cell migration [GO:1903977], positive regulation of substrate-dependent cell migration, cell attachment to substrate [GO:1904237], positive regulation of cell chemotaxis to fibroblast growth factor [GO:1904849], GO:1904859, GO:1905212, GO:1905312, positive regulation of mesenchymal stem cell migration [GO:1905322], positive regulation of hematopoietic stem cell migration [GO:2000473], positive regulation of metanephric mesenchymal cell migration [GO:2000591], GO:2001224 Definition: Any process that activates or increases the frequency, rate or extent of cell migration. Sources: GOC:go_curators Also known as: up regulation of cell migration, up-regulation of cell migration, upregulation of cell migration, activation of cell migration, stimulation of cell migration Relationships: is a type of regulation of cell migration [GO:0030334]; is a type of positive regulation of cell motility [GO:2000147]; positively regulates GO:0016477